{
  "term_label": "cell development",
  "gene": "UniProtKB:P78414",
  "gene_symbol": "IRX1",
  "term_id": "GO:0048468",
  "gene_name": "Iroquois-class homeodomain protein IRX-1"
}